{
  "term_label": "negative regulation of Ras protein signal transduction",
  "term_id": "GO:0046580",
  "gene_symbol": "LZTR1",
  "gene": "UniProtKB:Q8N653",
  "gene_name": "Leucine-zipper-like transcriptional regulator 1"
}